{
  "term_id": "GO:0016038",
  "term_label": "absorption of visible light",
  "gene": "UniProtKB:P04001",
  "gene_name": "Medium-wave-sensitive opsin 1",
  "gene_symbol": "OPN1MW"
}